inferior endocardial cushion morphogenesis [GO:1905317] (biological process) References: PMID:17050629 Sources: GOC:BHF, GOC:TermGenie, GOC:rl, GO_REF:0000083 Relationships: is a type of endocardial cushion morphogenesis [GO:0003203] Definition: The developmental process by which an inferior endocardial cushion is generated and organized. Also known as: ventral endocardial cushion morphogenesis